{
  "gene": "UniProtKB:Q96H86",
  "term_id": "GO:0006357",
  "term_label": "regulation of transcription by RNA polymerase II",
  "gene_symbol": "ZNF764",
  "gene_name": "Zinc finger protein 764"
}